regulation of lysosomal lumen pH [GO:0035751] (BP) Definition: Any process that modulates the pH of the lysosomal lumen, measured by the concentration of the hydrogen ion. Sources: GOC:rph Relationships: is a type of regulation of intracellular pH [GO:0051453]; is part of lysosome organization [GO:0007040] Subtypes: lysosomal lumen acidification [GO:0007042], lysosomal lumen pH elevation [GO:0035752]